{
  "gene_name": "Glycosyltransferase 1 domain-containing protein 1",
  "term_id": "UNKNOWN:0002",
  "gene": "UniProtKB:Q96MS3",
  "term_label": "Unknown biological process",
  "gene_symbol": "GLT1D1"
}